positive regulation of eosinophil differentiation [GO:0045645] (biological process) Definition: Any process that activates or increases the frequency, rate or extent of eosinophil differentiation. Relationships: is a type of positive regulation of granulocyte differentiation [GO:0030854]; is a type of GO:0045643; positively regulates eosinophil differentiation [GO:0030222] Sources: GOC:go_curators Also known as: up regulation of eosinophil differentiation, up-regulation of eosinophil differentiation, upregulation of eosinophil differentiation, activation of eosinophil differentiation, stimulation of eosinophil differentiation